{
  "term_label": "Unknown cellular component",
  "term_id": "UNKNOWN:0003",
  "gene": "UniProtKB:Q107X0",
  "gene_symbol": "KLKP1",
  "gene_name": "Putative protein KRIP1"
}